host intracellular region [GO:0043656] (cellular component) Relationships: is a type of GO:0033643 Sources: GOC:cc Definition: That space within the plasma membrane of a host cell. Also known as: host intracellular, intracellular region of host